{
  "term_id": "GO:0031616",
  "term_label": "spindle pole centrosome",
  "gene_symbol": "TBCCD1",
  "gene": "UniProtKB:Q9NVR7",
  "gene_name": "TBCC domain-containing protein 1"
}